{
  "gene": "UniProtKB:Q96DS6",
  "term_label": "Unknown molecular function",
  "gene_name": "Membrane-spanning 4-domains subfamily A member 6E",
  "gene_symbol": "MS4A6E",
  "term_id": "UNKNOWN:0001"
}